metanephric proximal convoluted tubule development [GO:0072229] (biological process) Relationships: is a type of proximal convoluted tubule development [GO:0072019]; is a type of metanephric nephron tubule development [GO:0072234]; is part of GO:0072237 Definition: The process whose specific outcome is the progression of the metanephric proximal convoluted tubule over time, from its formation to the mature structure. The metanephric proximal convoluted tubule is the most proximal portion of the metanephric proximal tubule and extends from the metanephric glomerular capsule to the metanephric proximal straight tubule. Sources: GOC:mtg_kidney_jan10